{
  "gene": "UniProtKB:P62166",
  "gene_name": "Neuronal calcium sensor 1",
  "gene_symbol": "NCS1",
  "term_label": "calcium sensitive guanylate cyclase activator activity",
  "term_id": "GO:0008048"
}